{
  "gene": "UniProtKB:Q9Y285",
  "gene_symbol": "FARSA",
  "term_id": "GO:0006432",
  "gene_name": "Phenylalanine--tRNA ligase alpha subunit",
  "term_label": "phenylalanyl-tRNA aminoacylation"
}